uridine nucleosidase activity [GO:0045437] (molecular function) Sources: EC:3.2.2.3, RHEA:15577 Also known as: uridine hydrolase activity, uridine ribohydrolase activity Definition: Catalysis of the reaction: H2O + uridine = ribofuranose + uracil. Relationships: is a type of ribosylpyrimidine nucleosidase activity [GO:0050263]